{
  "term_id": "GO:0005200",
  "term_label": "structural constituent of cytoskeleton",
  "gene_symbol": "ACTR1B",
  "gene": "UniProtKB:P42025",
  "gene_name": "Beta-centractin"
}